trans-Golgi network [GO:0005802] (cellular component) Also known as: trans face, TGN, trans Golgi network, Golgi trans face, Golgi trans-face, late Golgi, maturing face Definition: The network of interconnected tubular and cisternal structures located within the Golgi apparatus on the side distal to the endoplasmic reticulum, from which secretory vesicles emerge. The trans-Golgi network is important in the later stages of protein secretion where it is thought to play a key role in the sorting and targeting of secreted proteins to the correct destination. Note: There are different opinions about whether the TGN should be considered part of the Golgi apparatus or not. We follow Alberts et al, 1994 (ISBN:0815316194), who consider it to be a part. References: PMID:9695800 Sources: GOC:vw, ISBN:0815316194 Relationships: is a type of GO:0098791